{
  "gene_name": "cGMP-dependent protein kinase 1",
  "term_id": "UNKNOWN:0001",
  "term_label": "Unknown molecular function",
  "gene": "UniProtKB:Q13976",
  "gene_symbol": "PRKG1"
}